{
  "term_label": "extracellular region",
  "gene": "UniProtKB:O00584",
  "gene_symbol": "RNASET2",
  "term_id": "GO:0005576",
  "gene_name": "Ribonuclease T2"
}